{
  "gene_name": "Glycerophosphocholine cholinephosphodiesterase ENPP6",
  "gene_symbol": "ENPP6",
  "term_id": "GO:0006629",
  "term_label": "lipid metabolic process",
  "gene": "UniProtKB:Q6UWR7"
}